{
  "term_label": "Unknown cellular component",
  "gene": "UniProtKB:Q9NWL6",
  "gene_symbol": "ASNSD1",
  "term_id": "UNKNOWN:0003",
  "gene_name": "Asparagine synthetase domain-containing protein 1"
}